{
  "gene_name": "Interferon-induced transmembrane protein 1",
  "term_label": "response to interferon-beta",
  "gene": "UniProtKB:P13164",
  "term_id": "GO:0035456",
  "gene_symbol": "IFITM1"
}